{
  "gene_symbol": "SPANXN3",
  "term_label": "Unknown biological process",
  "gene": "UniProtKB:Q5MJ09",
  "term_id": "UNKNOWN:0002",
  "gene_name": "Sperm protein associated with the nucleus on the X chromosome N3"
}